{
  "gene_symbol": "DAP",
  "gene": "UniProtKB:P51397",
  "term_label": "Unknown cellular component",
  "gene_name": "Death-associated protein 1",
  "term_id": "UNKNOWN:0003"
}